Nsk1-Dlc1 complex [GO:0044816] (cellular component) Definition: A dimer of Nsk1 (nucleolus spindle kinetochore 1) and the dynein light chain, Dlc1. The dimers form an oligomeric chain structure. Functions in the regulation of kinetochore-microtubule interactions and chromosome segregation. Relationships: is a type of GO:0032991 References: PMID:22065639 Sources: GOC:vw